{
  "gene": "UniProtKB:O43462",
  "term_label": "regulation of response to endoplasmic reticulum stress",
  "term_id": "GO:1905897",
  "gene_name": "Membrane-bound transcription factor site-2 protease",
  "gene_symbol": "MBTPS2"
}